regulation of cytoskeleton polarization involved in growth plate cartilage chondrocyte division [GO:0003427] (biological process) Relationships: is a type of GO:0032878; is a type of regulation of cytoskeleton organization [GO:0051493]; is a type of Wnt signaling pathway, planar cell polarity pathway [GO:0060071]; regulates cytoskeleton polarization involved in growth plate cartilage chondrocyte division [GO:0003426] Definition: The series of molecular signals initiated by binding of a Wnt protein to a receptor on the surface of the target cell that modulates the rate, frequency, or extent of the polarization of cytoskeletal structures in a growth plate cartilage chondrocyte. This process results in the oriented division of the cell. Sources: GOC:ascb_2009, GOC:dph, GOC:tb Also known as: regulation of cytoskeleton polarization involved in growth plate cartilage chondrocyte division by planar cell polarity pathway